{
  "gene_name": "Coiled-coil domain-containing protein 71L",
  "gene_symbol": "CCDC71L",
  "term_id": "UNKNOWN:0002",
  "term_label": "Unknown biological process",
  "gene": "UniProtKB:Q8N9Z2"
}